{
  "gene": "UniProtKB:Q15428",
  "term_id": "GO:0071013",
  "term_label": "catalytic step 2 spliceosome",
  "gene_symbol": "SF3A2",
  "gene_name": "Splicing factor 3A subunit 2"
}